{
  "gene_symbol": "SLC23A3",
  "term_id": "UNKNOWN:0003",
  "gene_name": "Solute carrier family 23 member 3",
  "term_label": "Unknown cellular component",
  "gene": "UniProtKB:Q6PIS1"
}